{
  "gene_name": "Putative homeobox protein Meis3-like 2",
  "gene": "UniProtKB:A8K0S8",
  "term_label": "hemopoiesis",
  "term_id": "GO:0030097",
  "gene_symbol": "MEIS3P2"
}